beta-cyclopiazonate dehydrogenase activity [GO:0050448] (molecular function) Definition: Catalysis of the reaction: beta-cyclopiazonate + A = alpha-cyclopiazonate + AH(2). Sources: RHEA:14525 Also known as: b-cyclopiazonate dehydrogenase activity, beta-cyclopiazonate oxidocyclase activity, beta-cyclopiazonate:(acceptor) oxidoreductase (cyclizing), beta-cyclopiazonate:acceptor oxidoreductase (cyclizing), beta-cyclopiazonic oxidocyclase activity Relationships: is a type of oxidoreductase activity, acting on X-H and Y-H to form an X-Y bond [GO:0046992]